determination of stimulus location [GO:0050888] (biological process) Relationships: is_a sensory processing [GO:0050893] Definition: The determination of where on the body surface, within the body or in the environment a stimulus originates. Sources: ISBN:0721619908